{
  "term_id": "GO:0002523",
  "gene_symbol": "S100A9",
  "term_label": "leukocyte migration involved in inflammatory response",
  "gene_name": "Protein S100-A9",
  "gene": "UniProtKB:P06702"
}